negative regulation of N',N'',N'''-triacetylfusarinine C biosynthetic process [GO:1900696] (biological process) Sources: GOC:TermGenie, GOC:di Relationships: is a type of GO:1900377; is a type of GO:1900695; negatively regulates N',N'',N'''-triacetylfusarinine C biosynthetic process [GO:1900551] Also known as: down regulation of N',N'',N'''-triacetylfusarinine C anabolism, down regulation of N',N'',N'''-triacetylfusarinine C biosynthesis, down regulation of N',N'',N'''-triacetylfusarinine C biosynthetic process, down regulation of N',N'',N'''-triacetylfusarinine C formation, down regulation of N',N'',N'''-triacetylfusarinine C synthesis, down-regulation of N',N'',N'''-triacetylfusarinine C anabolism, down-regulation of N',N'',N'''-triacetylfusarinine C biosynthesis, down-regulation of N',N'',N'''-triacetylfusarinine C biosynthetic process, down-regulation of N',N'',N'''-triacetylfusarinine C formation, down-regulation of N',N'',N'''-triacetylfusarinine C synthesis, downregulation of N',N'',N'''-triacetylfusarinine C anabolism, downregulation of N',N'',N'''-triacetylfusarinine C biosynthesis, downregulation of N',N'',N'''-triacetylfusarinine C biosynthetic process, downregulation of N',N'',N'''-triacetylfusarinine C formation, downregulation of N',N'',N'''-triacetylfusarinine C synthesis, inhibition of N',N'',N'''-triacetylfusarinine C anabolism, inhibition of N',N'',N'''-triacetylfusarinine C biosynthesis, inhibition of N',N'',N'''-triacetylfusarinine C formation, inhibition of N',N'',N'''-triacetylfusarinine C synthesis, negative regulation of N',N'',N'''-triacetylfusarinine C anabolism, negative regulation of N',N'',N'''-triacetylfusarinine C biosynthesis, negative regulation of N',N'',N'''-triacetylfusarinine C formation, negative regulation of N',N'',N'''-triacetylfusarinine C synthesis, inhibition of N',N'',N'''-triacetylfusarinine C biosynthetic process Definition: Any process that stops, prevents or reduces the frequency, rate or extent of N',N'',N'''-triacetylfusarinine C biosynthetic process.